{
  "gene_name": "Peptidyl-prolyl cis-trans isomerase FKBP1C",
  "gene": "UniProtKB:Q5VVH2",
  "gene_symbol": "FKBP1C",
  "term_id": "GO:0033017",
  "term_label": "sarcoplasmic reticulum membrane"
}